regulation of ATP biosynthetic process [GO:2001169] (BP) Definition: Any process that modulates the frequency, rate or extent of ATP biosynthetic process. Sources: GOC:obol Also known as: regulation of ATP anabolism, regulation of ATP biosynthesis, regulation of ATP formation, regulation of ATP synthesis, regulation of ATP regeneration Relationships: is a type of GO:1900371; is a type of regulation of ATP metabolic process [GO:1903578]; regulates GO:0006754 Subtypes: GO:1905706, negative regulation of ATP biosynthetic process [GO:2001170], positive regulation of ATP biosynthetic process [GO:2001171]